{
  "gene_name": "Splicing regulator ARVCF",
  "gene": "UniProtKB:O00192",
  "term_id": "GO:0005737",
  "term_label": "cytoplasm",
  "gene_symbol": "ARVCF"
}